{
  "term_label": "nucleus",
  "gene": "UniProtKB:Q02086",
  "term_id": "GO:0005634",
  "gene_name": "Transcription factor Sp2",
  "gene_symbol": "SP2"
}